{
  "gene": "UniProtKB:Q86TU6",
  "gene_name": "Putative uncharacterized protein encoded by LINC00523",
  "term_label": "Unknown biological process",
  "term_id": "UNKNOWN:0002",
  "gene_symbol": "LINC00523"
}